{
  "term_label": "SCF ubiquitin ligase complex",
  "term_id": "GO:0019005",
  "gene_symbol": "FBXO9",
  "gene_name": "F-box only protein 9",
  "gene": "UniProtKB:Q9UK97"
}